{
  "gene_name": "Cancer-associated gene 1 protein",
  "gene_symbol": "CAGE1",
  "term_id": "UNKNOWN:0001",
  "gene": "UniProtKB:Q8TC20",
  "term_label": "Unknown molecular function"
}